{
  "term_label": "regulation of protein stability",
  "term_id": "GO:0031647",
  "gene_symbol": "USP17L2",
  "gene": "UniProtKB:Q6R6M4",
  "gene_name": "Ubiquitin carboxyl-terminal hydrolase 17"
}